trimethylenediamine catabolic process [GO:1901056] (biological process) Definition: The chemical reactions and pathways resulting in the breakdown of trimethylenediamine. Relationships: is a type of GO:0006598 Sources: GOC:TermGenie, GOC:yaf, UniPathway:UPA00010 Also known as: trimethylenediamine breakdown, trimethylenediamine catabolism, trimethylenediamine degradation